negative regulation of antigen processing and presentation via MHC class Ib [GO:0002593] (biological process) Subtypes: negative regulation of antigen processing and presentation of peptide antigen via MHC class Ib [GO:0002596], negative regulation of antigen processing and presentation of lipid antigen via MHC class Ib [GO:0002599] Sources: GOC:add Also known as: down regulation of antigen processing and presentation via MHC class Ib, down-regulation of antigen processing and presentation via MHC class Ib, downregulation of antigen processing and presentation via MHC class Ib, inhibition of antigen processing and presentation via MHC class Ib Definition: Any process that stops, prevents, or reduces the frequency, rate, or extent of antigen processing and presentation of antigen via MHC class Ib. Relationships: is a type of negative regulation of antigen processing and presentation [GO:0002578]; is a type of regulation of antigen processing and presentation via MHC class Ib [GO:0002592]; negatively regulates antigen processing and presentation via MHC class Ib [GO:0002475]